{
  "term_id": "GO:0007155",
  "gene": "UniProtKB:P16591",
  "gene_symbol": "FER",
  "term_label": "cell adhesion",
  "gene_name": "Tyrosine-protein kinase Fer"
}